{
  "term_id": "GO:0005737",
  "term_label": "cytoplasm",
  "gene_symbol": "ZRANB1",
  "gene": "UniProtKB:Q9UGI0",
  "gene_name": "Ubiquitin thioesterase ZRANB1"
}